{
  "gene_symbol": "BEST4",
  "gene_name": "Bestrophin-4",
  "term_label": "chloride transmembrane transport",
  "term_id": "GO:1902476",
  "gene": "UniProtKB:Q8NFU0"
}